{
  "term_label": "cytoplasm",
  "gene": "UniProtKB:Q96GX9",
  "gene_symbol": "APIP",
  "term_id": "GO:0005737",
  "gene_name": "Methylthioribulose-1-phosphate dehydratase"
}